acetylcholine transport [GO:0015870] (biological process) Relationships: is a type of organic cation transport [GO:0015695]; is a type of nitrogen compound transport [GO:0071705]; is_a GO:1901374 Definition: The directed movement of acetylcholine into, out of or within a cell, or between cells, by means of some agent such as a transporter or pore. Acetylcholine is an acetic acid ester of the organic base choline and functions as a neurotransmitter, released at the synapses of parasympathetic nerves and at neuromuscular junctions. Sources: GOC:ai Subtypes: GO:0051630, acetylcholine secretion [GO:0061526]